{
  "term_label": "oxidoreductase activity, acting on single donors with incorporation of molecular oxygen, incorporation of two atoms of oxygen",
  "gene_symbol": "PTGS1",
  "gene_name": "Prostaglandin G_H synthase 1",
  "term_id": "GO:0016702",
  "gene": "UniProtKB:P23219"
}